{
  "gene_symbol": "HOMER2",
  "gene_name": "Homer protein homolog 2",
  "term_label": "cytoplasm",
  "term_id": "GO:0005737",
  "gene": "UniProtKB:Q9NSB8"
}